lung epithelium development [GO:0060428] (biological process) Relationships: is_a GO:0060429; is part of lung development [GO:0030324] Also known as: pulmonary epithelium development Subtypes: lobar bronchus epithelium development [GO:0060481], alveolar primary septum development [GO:0061143], GO:0061144 Definition: The biological process whose specific outcome is the progression of the lung epithelium from an initial condition to its mature state. This process begins with the formation of lung epithelium and ends with the mature structure. The lung epithelium is the specialized epithelium that lines the inside of the lung. Sources: GOC:dph, GOC:mtg_lung